{
  "gene_name": "Microtubule-associated protein 1B",
  "gene_symbol": "MAP1B",
  "term_id": "GO:0031114",
  "term_label": "regulation of microtubule depolymerization",
  "gene": "UniProtKB:P46821"
}